mRNA cap binding complex binding [GO:0140262] (molecular function) Definition: Binding to a mRNA cap binding complex. References: PMID:16938833 Relationships: is a type of protein-containing complex binding [GO:0044877]